{
  "term_id": "GO:0043330",
  "gene_symbol": "IFNA8",
  "term_label": "response to exogenous dsRNA",
  "gene": "UniProtKB:P32881",
  "gene_name": "Interferon alpha-8"
}